{
  "term_label": "phosphatidylinositol-mediated signaling",
  "gene": "UniProtKB:Q4KWH8",
  "term_id": "GO:0048015",
  "gene_name": "1-phosphatidylinositol 4,5-bisphosphate phosphodiesterase eta-1",
  "gene_symbol": "PLCH1"
}